{
  "term_label": "Unknown biological process",
  "gene": "UniProtKB:Q7Z736",
  "gene_symbol": "PLEKHH3",
  "term_id": "UNKNOWN:0002",
  "gene_name": "Pleckstrin homology domain-containing family H member 3"
}